{
  "gene_name": "Paraneoplastic antigen-like protein 5",
  "term_label": "Unknown cellular component",
  "gene": "UniProtKB:Q96PV4",
  "term_id": "UNKNOWN:0003",
  "gene_symbol": "PNMA5"
}